{
  "gene_symbol": "DNTTIP2",
  "term_id": "UNKNOWN:0001",
  "gene": "UniProtKB:Q5QJE6",
  "gene_name": "Deoxynucleotidyltransferase terminal-interacting protein 2",
  "term_label": "Unknown molecular function"
}